{
  "gene_symbol": "CHRM2",
  "term_id": "GO:0007197",
  "gene_name": "Muscarinic acetylcholine receptor M2",
  "term_label": "adenylate cyclase-inhibiting G protein-coupled acetylcholine receptor signaling pathway",
  "gene": "UniProtKB:P08172"
}